{
  "gene_symbol": "MYCL",
  "gene": "UniProtKB:P12524",
  "gene_name": "Protein L-Myc",
  "term_label": "Unknown cellular component",
  "term_id": "UNKNOWN:0003"
}